negative regulation of gastro-intestinal system smooth muscle contraction [GO:1904305] (BP) Relationships: is_a negative regulation of smooth muscle contraction [GO:0045986]; is a type of regulation of gastro-intestinal system smooth muscle contraction [GO:1904304]; negatively regulates GO:0014831 Subtypes: negative regulation of stomach fundus smooth muscle contraction [GO:0120070], negative regulation of pyloric antrum smooth muscle contraction [GO:0120073], GO:1904342, negative regulation of small intestine smooth muscle contraction [GO:1904348] Also known as: down regulation of gastro-intestinal system smooth muscle contraction, down-regulation of gastro-intestinal system smooth muscle contraction, downregulation of gastro-intestinal system smooth muscle contraction, inhibition of gastro-intestinal system smooth muscle contraction Definition: Any process that stops, prevents or reduces the frequency, rate or extent of gastro-intestinal system smooth muscle contraction. References: PMID:10821044 Sources: GOC:TermGenie, GO_REF:0000058